{
  "gene": "UniProtKB:Q7L7X3",
  "gene_symbol": "TAOK1",
  "gene_name": "Serine_threonine-protein kinase TAO1",
  "term_id": "GO:0005737",
  "term_label": "cytoplasm"
}